{
  "gene_name": "Myosin-1",
  "gene_symbol": "MYH1",
  "term_label": "actin filament binding",
  "gene": "UniProtKB:P12882",
  "term_id": "GO:0051015"
}